negative regulation of L-leucine biosynthetic process [GO:2001277] (biological process) Also known as: negative regulation of leucine biosynthetic process, negative regulation of L-leucine anabolism, negative regulation of L-leucine biosynthesis, negative regulation of L-leucine formation, negative regulation of L-leucine synthesis Relationships: is a type of GO:0062014; is_a GO:2000283; is a type of regulation of L-leucine biosynthetic process [GO:2001276]; RO_0002212 GO:0009098 Definition: Any process that stops, prevents or reduces the frequency, rate or extent of L-leucine biosynthetic process. Sources: GOC:obol